{
  "term_label": "flagellated sperm motility",
  "gene_symbol": "IQUB",
  "gene_name": "IQ and ubiquitin-like domain-containing protein",
  "gene": "UniProtKB:Q8NA54",
  "term_id": "GO:0030317"
}